{
  "term_id": "GO:0098632",
  "gene_name": "Cell adhesion molecule DSCAM",
  "gene_symbol": "DSCAM",
  "term_label": "cell-cell adhesion mediator activity",
  "gene": "UniProtKB:O60469"
}